{
  "gene": "UniProtKB:P30530",
  "gene_name": "Tyrosine-protein kinase receptor UFO",
  "term_label": "transmembrane receptor protein tyrosine kinase activity",
  "term_id": "GO:0004714",
  "gene_symbol": "AXL"
}